cephalic furrow formation [GO:0007376] (biological process) Sources: ISBN:0879694238 Relationships: is_a anatomical structure formation involved in morphogenesis [GO:0048646]; is part of gastrulation involving germ band extension [GO:0010004] Definition: Formation of a partial necklace of inturning tissue on the lateral sides of the embryo, along the dorsal-ventral axis. This furrow demarcates head from thorax in the developing protostome.